{
  "term_id": "GO:0008081",
  "term_label": "phosphoric diester hydrolase activity",
  "gene_name": "PI-PLC X domain-containing protein 3",
  "gene": "UniProtKB:Q63HM9",
  "gene_symbol": "PLCXD3"
}